{
  "gene_symbol": "CDK5R1",
  "gene_name": "Cyclin-dependent kinase 5 activator 1",
  "gene": "UniProtKB:Q15078",
  "term_id": "GO:0019901",
  "term_label": "protein kinase binding"
}